{
  "gene_name": "Midnolin",
  "term_label": "Unknown biological process",
  "gene_symbol": "MIDN",
  "gene": "UniProtKB:Q504T8",
  "term_id": "UNKNOWN:0002"
}